{
  "gene_symbol": "CCAR2",
  "term_id": "UNKNOWN:0003",
  "term_label": "Unknown cellular component",
  "gene": "UniProtKB:Q8N163",
  "gene_name": "Cell cycle and apoptosis regulator protein 2"
}